establishment of left/right asymmetry [GO:0061966] (biological process) Definition: The initial formation of the type asymmetry in an organism's body plan or part of an organism with respect to the left and right halves. Relationships: is a type of determination of left/right symmetry [GO:0007368] References: PMID:18629866 Sources: GOC:BHF Subtypes: establishment of left sidedness [GO:0061967]